{
  "gene": "UniProtKB:Q6ZMI0",
  "gene_symbol": "PPP1R21",
  "term_label": "Unknown biological process",
  "gene_name": "Protein phosphatase 1 regulatory subunit 21",
  "term_id": "UNKNOWN:0002"
}